{
  "term_label": "regulation of transcription by RNA polymerase II",
  "gene_symbol": "MSX1",
  "gene_name": "Homeobox protein MSX-1",
  "gene": "UniProtKB:P28360",
  "term_id": "GO:0006357"
}